tumor necrosis factor receptor binding [GO:0005164] (molecular function) Sources: GOC:ai Relationships: is a type of tumor necrosis factor receptor superfamily binding [GO:0032813] Also known as: TNF receptor binding, tumor necrosis factor, tumor necrosis factor receptor ligand Definition: Binding to a tumor necrosis factor receptor.